mitochondrion migration along actin filament [GO:0034642] (biological process) References: PMID:15979253, PMID:16306220 Sources: GOC:mah Definition: The directed movement of a mitochondrion along a microfilament, mediated by motor proteins. Also known as: mitochondrial migration along actin filament, mitochondrial migration along microfilament, mitochondrial migration, actin-mediated, mitochondrion migration along microfilament, mitochondrion transport along actin filament Relationships: is_a GO:0030048; is a type of establishment of mitochondrion localization [GO:0051654]; is a type of GO:0099515